{
  "term_label": "nucleus",
  "gene_symbol": "ZNF569",
  "gene": "UniProtKB:Q5MCW4",
  "gene_name": "Zinc finger protein 569",
  "term_id": "GO:0005634"
}